{
  "term_id": "GO:0005667",
  "gene": "UniProtKB:P15923",
  "gene_symbol": "TCF3",
  "term_label": "transcription regulator complex",
  "gene_name": "Transcription factor E2-alpha"
}